{
  "gene_symbol": "INKA2",
  "gene_name": "PAK4-inhibitor INKA2",
  "term_label": "Unknown biological process",
  "gene": "UniProtKB:Q9NTI7",
  "term_id": "UNKNOWN:0002"
}